{
  "term_label": "stereocilium maintenance",
  "term_id": "GO:0120045",
  "gene": "UniProtKB:Q4KMQ1",
  "gene_name": "Taperin",
  "gene_symbol": "TPRN"
}